phosphatidylinositol 4-phosphate biosynthetic process [GO:0180048] (biological process) Definition: The chemical reactions and pathways resulting in the formation of phosphatidylinositol 4-phosphate. Relationships: is a type of biosynthetic process [GO:0009058] Also known as: 1-phosphatidyl-1D-myo-inositol 4-phosphate biosynthesis, 1-phosphatidyl-1D-myo-inositol biosynthetic process, PI4P biosynthesis, phosphatidylinositol (PI)-4- phosphate biosynthetic process, phosphatidylinositol-4-phosphate synthesis References: PMID:39239853